{
  "term_label": "nucleus",
  "term_id": "GO:0005634",
  "gene_symbol": "L3MBTL1",
  "gene": "UniProtKB:Q9Y468",
  "gene_name": "Lethal(3)malignant brain tumor-like protein 1"
}